9-cis-retinoic acid biosynthetic process [GO:0042904] (biological process) Relationships: is a type of retinoic acid biosynthetic process [GO:0002138]; is a type of 9-cis-retinoic acid metabolic process [GO:0042905] Also known as: 9-cis-retinoic acid anabolism, 9-cis-retinoic acid biosynthesis, 9-cis-retinoic acid formation, 9-cis-retinoic acid synthesis Definition: The chemical reactions and pathways resulting in the formation of 9-cis-retinoic acid, a metabolically active vitamin A derivative. References: PMID:11279029 Sources: GOC:jl